positive regulation of phenotypic switching [GO:1900241] (biological process) Relationships: is a type of GO:0048522; is a type of regulation of phenotypic switching [GO:1900239]; positively regulates GO:0036166 Definition: Any process that activates or increases the frequency, rate or extent of phenotypic switching. Also known as: up regulation of phenotypic switching, up-regulation of phenotypic switching, upregulation of phenotypic switching, activation of phenotypic switching, activation of phenotypic dimorphism, positive regulation of phenotypic dimorphism, up regulation of phenotypic dimorphism, up-regulation of phenotypic dimorphism, upregulation of phenotypic dimorphism Sources: GOC:TermGenie, GOC:di